{
  "term_id": "GO:0006355",
  "gene": "UniProtKB:Q8N488",
  "gene_name": "RING1 and YY1-binding protein",
  "term_label": "regulation of DNA-templated transcription",
  "gene_symbol": "RYBP"
}